{
  "gene_name": "Inactive dipeptidyl peptidase 10",
  "term_label": "voltage-gated potassium channel complex",
  "gene": "UniProtKB:Q8N608",
  "gene_symbol": "DPP10",
  "term_id": "GO:0008076"
}